{
  "gene_symbol": "NRBP2",
  "term_id": "GO:0035556",
  "gene": "UniProtKB:Q9NSY0",
  "gene_name": "Nuclear receptor-binding protein 2",
  "term_label": "intracellular signal transduction"
}